indolepyruvate C-methyltransferase activity [GO:0030747] (molecular function) Sources: EC:2.1.1.47 Definition: Catalysis of the reaction: indole-3-pyruvate + S-adenosyl-L-methionine = (R)-3-(indol-3-yl)-2-oxobutanoate + H+ + S-adenosyl-L-homocysteine. Relationships: is a type of S-adenosylmethionine-dependent methyltransferase activity [GO:0008757] Also known as: S-adenosyl-L-methionine:(indol-3-yl)pyruvate C-methyltransferase activity, S-adenosyl-L-methionine:indolepyruvate C-methyltransferase activity, indolepyruvate 3-methyltransferase activity, indolepyruvate methyltransferase activity, indolepyruvic acid methyltransferase activity